{
  "gene": "UniProtKB:O75116",
  "gene_symbol": "ROCK2",
  "gene_name": "Rho-associated protein kinase 2",
  "term_id": "GO:0032956",
  "term_label": "regulation of actin cytoskeleton organization"
}